{
  "gene_symbol": "RAB37",
  "gene": "UniProtKB:Q96AX2",
  "term_id": "GO:0005768",
  "gene_name": "Ras-related protein Rab-37",
  "term_label": "endosome"
}